mRNA cis splicing, via spliceosome [GO:0045292] (biological process) Regulation: regulated by regulation of mRNA cis splicing, via spliceosome [GO:1905744]; negatively regulated by negative regulation of mRNA cis splicing, via spliceosome [GO:1905745]; positively regulated by positive regulation of mRNA cis splicing, via spliceosome [GO:1905746] Definition: The joining together, after removal of an intervening sequence composed of one or more introns, of two segments of the same RNA molecule via spliceosomal catalysis to produce an mRNA composed only of exon sequences that all came from the same primary transcript. References: PMID:18458335 Sources: GOC:krc, ISBN:0879695897 Also known as: splicing, nuclear mRNA cis splicing, via spliceosome, nuclear mRNA cis splicing, via U2-type spliceosome Relationships: is a type of GO:0000398